{
  "term_id": "GO:0070498",
  "gene_name": "Interleukin-1 receptor-associated kinase 1",
  "term_label": "interleukin-1-mediated signaling pathway",
  "gene": "UniProtKB:P51617",
  "gene_symbol": "IRAK1"
}